biological process involved in intraspecies interaction between organisms [GO:0051703] (biological process) Definition: Any process in which an organism has an effect on an organism of the same species. Relationships: is a type of biological_process [GO:0008150] Sources: GOC:ai Subtypes: flocculation [GO:0000128], agglutination involved in conjugation with cellular fusion [GO:0000752], agglutination involved in conjugation with mutual genetic exchange [GO:0000758], pollen tube adhesion [GO:0009865], pollen tube reception [GO:0010483], social behavior [GO:0035176], GO:0044010, socially cooperative development [GO:0099120], olfactory sociosexual communication [GO:0120318] Also known as: intraspecies interaction between organisms, intraspecies interaction with other organisms